regulation of cell division [GO:0051302] (biological process) Definition: Any process that modulates the frequency, rate or extent of the physical partitioning and separation of a cell into daughter cells. Sources: GOC:go_curators Relationships: is a type of GO:0050794; regulates cell division [GO:0051301] Subtypes: regulation of cell budding [GO:0007116], regulation of asymmetric cell division [GO:0009786], GO:0010482, regulation of cytokinesis [GO:0032465], GO:0051781, negative regulation of cell division [GO:0051782], GO:2000035